{
  "gene": "UniProtKB:Q9BYJ4",
  "gene_name": "E3 ubiquitin-protein ligase TRIM34",
  "gene_symbol": "TRIM34",
  "term_label": "innate immune response",
  "term_id": "GO:0045087"
}